monoatomic ion antiporter activity involved in regulation of postsynaptic membrane potential [GO:0099580] (molecular function) Definition: Any ion antiporter activity, occurring in the postsynaptic membrane, that is involved in regulation of postsynaptic membrane potential. Sources: GOC:dos Also known as: ion antiporter activity involved in regulation of post-synaptic membrane potential, ion antiporter activity involved in regulation of postsynaptic membrane potential Relationships: is a type of GO:0015297; occurs in postsynaptic membrane [GO:0045211]